{
  "term_label": "ubiquitin protein ligase activity",
  "gene_name": "E3 ubiquitin-protein ligase ARK2C",
  "gene_symbol": "ARK2C",
  "gene": "UniProtKB:Q6ZSG1",
  "term_id": "GO:0061630"
}